{
  "gene": "UniProtKB:Q9BTC8",
  "gene_symbol": "MTA3",
  "term_id": "GO:0005654",
  "term_label": "nucleoplasm",
  "gene_name": "Metastasis-associated protein MTA3"
}